{
  "gene": "UniProtKB:P49279",
  "term_id": "GO:0005384",
  "term_label": "manganese ion transmembrane transporter activity",
  "gene_symbol": "SLC11A1",
  "gene_name": "Natural resistance-associated macrophage protein 1"
}